receptor diffusion trapping [GO:0098953] (biological process) Subtypes: neurotransmitter receptor diffusion trapping [GO:0099628] References: PMID:18832033 Definition: The process by which a membrane receptor, diffusing freely within the plasma membeane, becomes trapped in some plasma membrane region. This can happen when a receptor bind, directly or indirectly, to some component of the underlying matrix. Relationships: is a type of localization within membrane [GO:0051668]; occurs in GO:0005886